{
  "gene_symbol": "NDUFA7",
  "gene_name": "NADH dehydrogenase [ubiquinone] 1 alpha subcomplex subunit 7",
  "gene": "UniProtKB:O95182",
  "term_label": "respiratory chain complex I",
  "term_id": "GO:0045271"
}